negative regulation of lipid localization [GO:1905953] (biological process) Definition: Any process that stops, prevents or reduces the frequency, rate or extent of lipid localization. References: PMID:17564681 Sources: GOC:TermGenie, GO_REF:0000058 Also known as: down regulation of lipid localisation, down regulation of lipid localization, down-regulation of lipid localisation, down-regulation of lipid localization, downregulation of lipid localisation, downregulation of lipid localization, negative regulation of lipid localisation, inhibition of lipid localisation, inhibition of lipid localization Relationships: is a type of negative regulation of biological process [GO:0048519]; is_a GO:1905952; negatively regulates GO:0010876 Subtypes: negative regulation of lipid storage [GO:0010888], negative regulation of lipid transport [GO:0032369]